{
  "term_label": "nucleoplasm",
  "gene": "UniProtKB:Q5THR3",
  "term_id": "GO:0005654",
  "gene_name": "EF-hand calcium-binding domain-containing protein 6",
  "gene_symbol": "EFCAB6"
}